{
  "term_id": "GO:0031490",
  "gene_symbol": "SUZ12",
  "gene": "UniProtKB:Q15022",
  "term_label": "chromatin DNA binding",
  "gene_name": "Polycomb protein SUZ12"
}